{
  "gene_symbol": "HLA-DRB4",
  "gene": "UniProtKB:P13762",
  "gene_name": "HLA class II histocompatibility antigen, DR beta 4 chain",
  "term_label": "peptide antigen assembly with MHC class II protein complex",
  "term_id": "GO:0002503"
}